{
  "term_label": "L-glutamine transmembrane transporter activity",
  "gene_name": "Sodium-coupled neutral amino acid symporter 2",
  "gene_symbol": "SLC38A2",
  "term_id": "GO:0015186",
  "gene": "UniProtKB:Q96QD8"
}